{
  "gene_name": "Leukocyte tyrosine kinase receptor",
  "gene": "UniProtKB:P29376",
  "term_label": "receptor complex",
  "gene_symbol": "LTK",
  "term_id": "GO:0043235"
}